{
  "term_label": "intra-Golgi vesicle-mediated transport",
  "gene_symbol": "COG2",
  "gene": "UniProtKB:Q14746",
  "gene_name": "Conserved oligomeric Golgi complex subunit 2",
  "term_id": "GO:0006891"
}